neuron projection organization [GO:0106027] (biological process) Definition: A process that is carried out at the cellular level which results in the assembly, arrangement of constituent parts, or disassembly of a prolongation or process extending from a neuron, e.g. an axon, or a dendrite. Relationships: is a type of plasma membrane bounded cell projection organization [GO:0120036] References: PMID:11585923 Sources: GOC:aruk, GOC:bc Subtypes: vestibular receptor cell stereocilium organization [GO:0060121], dendritic spine organization [GO:0097061], neuron projection retraction [GO:0106028], neuron projection maintenance [GO:1990535]